{
  "gene_name": "UAP56-interacting factor",
  "gene": "UniProtKB:Q96QD9",
  "term_id": "GO:0003729",
  "gene_symbol": "FYTTD1",
  "term_label": "mRNA binding"
}